{
  "term_id": "GO:0005938",
  "gene_symbol": "FRYL",
  "term_label": "cell cortex",
  "gene": "UniProtKB:O94915",
  "gene_name": "Protein furry homolog-like"
}